isoleucine-tRNA ligase activity [GO:0004822] (MF) Also known as: isoleucyl-tRNA synthetase activity, L-isoleucine:tRNAIle ligase (AMP-forming), isoleucine translase activity, isoleucine-tRNA synthetase activity, isoleucine-transfer RNA ligase activity, isoleucyl-transfer RNA synthetase activity, isoleucyl-transfer ribonucleate synthetase activity Definition: Catalysis of the reaction: L-isoleucine + ATP + tRNA(Ile) = L-isoleucyl-tRNA(Ile) + AMP + diphosphate + 2 H+. Sources: EC:6.1.1.5, RHEA:11060 Relationships: is_a aminoacyl-tRNA ligase activity [GO:0004812]